{
  "gene": "UniProtKB:Q8IVH4",
  "gene_name": "Methylmalonic aciduria type A protein, mitochondrial",
  "gene_symbol": "MMAA",
  "term_label": "Unknown biological process",
  "term_id": "UNKNOWN:0002"
}